transporter regulator activity [GO:0141108] (molecular function) Relationships: is a type of GO:0098772; regulates transporter activity [GO:0005215] Sources: GOC:curators Subtypes: channel regulator activity [GO:0016247], transporter activator activity [GO:0141109], transporter inhibitor activity [GO:0141110] Definition: Binds to and modulates the activity of a transporter.